defense response to parasitic plant [GO:0002242] (biological process) Definition: Reactions triggered in response to the presence of a parasitic plant that act to protect an organism. Sources: GOC:add Relationships: is a type of response to parasitic plant [GO:0002241]; is a type of defense response to other organism [GO:0098542]